protein de-2-hydroxyisobutyrylase activity [GO:0160010] (molecular function) Definition: Catalysis of the reaction: H2O + N6-(2-hydroxyisobutanoyl)-L-lysyl-[protein] = 2-hydroxy-2-methylpropanoate + L-lysyl-[protein]. References: PMID:29192674 Relationships: is a type of hydrolase activity, acting on carbon-nitrogen (but not peptide) bonds, in linear amides [GO:0016811]